{
  "term_label": "fatty acid biosynthetic process",
  "gene_name": "Acyl-coenzyme A synthetase ACSM6, mitochondrial",
  "gene_symbol": "ACSM6",
  "term_id": "GO:0006633",
  "gene": "UniProtKB:Q6P461"
}